{
  "gene_name": "Uncharacterized protein",
  "gene": "UniProtKB:A0A7I2V2S6",
  "gene_symbol": "A0A7I2V2S6",
  "term_id": "UNKNOWN:0001",
  "term_label": "Unknown molecular function"
}